{
  "gene_name": "Synaptosomal-associated protein 47",
  "term_label": "SNAP receptor activity",
  "gene_symbol": "SNAP47",
  "gene": "UniProtKB:Q5SQN1",
  "term_id": "GO:0005484"
}